negative regulation of nematode male tail tip morphogenesis [GO:0110038] (biological process) Definition: Any process that stops, prevents, or reduces the frequency, rate or extent of nematode male tail tip morphogenesis. Relationships: is a type of negative regulation of developmental process [GO:0051093]; is a type of negative regulation of multicellular organismal process [GO:0051241]; is_a regulation of nematode male tail tip morphogenesis [GO:0110037]; negatively regulates nematode male tail tip morphogenesis [GO:0045138] References: PMID:28068334 Sources: GOC:rz